{
  "term_label": "Unknown cellular component",
  "gene": "UniProtKB:A8MVA2",
  "term_id": "UNKNOWN:0003",
  "gene_name": "Keratin-associated protein 9-6",
  "gene_symbol": "KRTAP9-6"
}